{
  "gene_symbol": "PPP1R3D",
  "gene": "UniProtKB:O95685",
  "term_label": "glycogen binding",
  "term_id": "GO:2001069",
  "gene_name": "Protein phosphatase 1 regulatory subunit 3D"
}